{
  "gene_name": "Immunoglobulin subtype domain-containing protein",
  "term_id": "GO:0140375",
  "gene": "UniProtKB:A0A1W2PRS3",
  "gene_symbol": "A0A1W2PRS3",
  "term_label": "immune receptor activity"
}